{
  "term_label": "signaling receptor binding",
  "gene": "UniProtKB:Q99944",
  "term_id": "GO:0005102",
  "gene_name": "Epidermal growth factor-like protein 8",
  "gene_symbol": "EGFL8"
}